{
  "term_id": "GO:0005829",
  "gene_symbol": "NQO2",
  "term_label": "cytosol",
  "gene_name": "Ribosyldihydronicotinamide dehydrogenase [quinone]",
  "gene": "UniProtKB:P16083"
}